{
  "term_label": "neuron differentiation",
  "gene_symbol": "WNT7B",
  "gene": "UniProtKB:P56706",
  "term_id": "GO:0030182",
  "gene_name": "Protein Wnt-7b"
}